{
  "gene_symbol": "DMRTB1",
  "term_id": "GO:0000981",
  "gene_name": "Doublesex- and mab-3-related transcription factor B1",
  "term_label": "DNA-binding transcription factor activity, RNA polymerase II-specific",
  "gene": "UniProtKB:Q96MA1"
}